{
  "gene_symbol": "NF2",
  "gene": "UniProtKB:P35240",
  "gene_name": "Merlin",
  "term_id": "GO:2000643",
  "term_label": "positive regulation of early endosome to late endosome transport"
}